{
  "gene": "UniProtKB:P62491",
  "term_id": "GO:0030133",
  "gene_symbol": "RAB11A",
  "gene_name": "Ras-related protein Rab-11A",
  "term_label": "transport vesicle"
}